{
  "gene": "UniProtKB:Q9Y2Y0",
  "gene_name": "ADP-ribosylation factor-like protein 2-binding protein",
  "term_label": "Unknown molecular function",
  "term_id": "UNKNOWN:0001",
  "gene_symbol": "ARL2BP"
}